{
  "gene": "UniProtKB:Q68D51",
  "term_id": "UNKNOWN:0001",
  "gene_name": "DENN domain-containing protein 2C",
  "gene_symbol": "DENND2C",
  "term_label": "Unknown molecular function"
}